{
  "term_id": "GO:0000785",
  "gene_symbol": "KDM3B",
  "gene_name": "Lysine-specific demethylase 3B",
  "term_label": "chromatin",
  "gene": "UniProtKB:Q7LBC6"
}